{
  "gene_name": "E3 ubiquitin-protein ligase TRIM58",
  "term_label": "regulation of gene expression",
  "gene": "UniProtKB:Q8NG06",
  "term_id": "GO:0010468",
  "gene_symbol": "TRIM58"
}